{
  "term_label": "RNA polymerase II cis-regulatory region sequence-specific DNA binding",
  "gene_symbol": "ZNF649",
  "term_id": "GO:0000978",
  "gene": "UniProtKB:Q9BS31",
  "gene_name": "Zinc finger protein 649"
}